{
  "term_id": "UNKNOWN:0002",
  "gene": "UniProtKB:Q96P15",
  "gene_name": "Serpin B11",
  "term_label": "Unknown biological process",
  "gene_symbol": "SERPINB11"
}